{
  "term_label": "plasma membrane",
  "term_id": "GO:0005886",
  "gene_symbol": "MS4A5",
  "gene_name": "Membrane-spanning 4-domains subfamily A member 5",
  "gene": "UniProtKB:Q9H3V2"
}